{
  "term_id": "GO:0031424",
  "term_label": "keratinization",
  "gene_symbol": "KRT85",
  "gene": "UniProtKB:P78386",
  "gene_name": "Keratin, type II cuticular Hb5"
}